{
  "term_id": "GO:0045944",
  "term_label": "positive regulation of transcription by RNA polymerase II",
  "gene_symbol": "PCBP2",
  "gene_name": "Poly(rC)-binding protein 2",
  "gene": "UniProtKB:Q15366"
}